IgA immunoglobulin complex [GO:0071745] (cellular component) Note: Note that an IgA immunoglobulin complex has the function of antigen binding if a suitable antigen is available. Definition: A protein complex composed of two identical immunoglobulin heavy chains of the IgA isotype and two identical immunoglobulin light chains, held together by disulfide bonds, and sometimes complexed with J chain or J chain and secretory component. An IgA immunoglobulin complex may be embedded in the plasma membrane or present in the extracellular space, in mucosal areas or other tissues, or circulating in the blood or lymph. Subtypes: IgA immunoglobulin complex, circulating [GO:0071746], IgA B cell receptor complex [GO:0071747] References: PMID:16362985 Sources: GOC:add, ISBN:0781765196 Also known as: IgA1 antibody, IgA2 antibody Relationships: is a type of immunoglobulin complex [GO:0019814]